{
  "gene_symbol": "FAM107A",
  "gene_name": "Actin-associated protein FAM107A",
  "term_label": "Unknown molecular function",
  "term_id": "UNKNOWN:0001",
  "gene": "UniProtKB:O95990"
}